antigen processing and presentation of exogenous protein antigen via MHC class Ib, TAP-dependent [GO:0002481] (biological process) Relationships: is a type of antigen processing and presentation of exogenous peptide antigen via MHC class Ib [GO:0002477] Also known as: TAP-dependent antigen processing and presentation of exogenous peptide antigen via MHC class Ib, TAP-dependent exogenous peptide antigen processing and presentation via MHC class Ib, exogenous peptide antigen processing and presentation via MHC class Ib, TAP-dependent Definition: The process in which an antigen-presenting cell expresses a peptide antigen of exogenous origin on its cell surface in association with an MHC class Ib protein complex following intracellular transport via a TAP (transporter associated with antigen processing) pathway. The peptide is typically a fragment of a larger exogenous protein which has been degraded within the cell and is dependent on TAP transport from the cytosol to ER for association with the MHC class Ib molecule. Class Ib here refers to non-classical class I molecules, such as those of the HLA-E gene family. References: PMID:15928678 Sources: GOC:add